{
  "term_id": "UNKNOWN:0002",
  "gene_symbol": "MINDY4B",
  "gene": "UniProtKB:A8MYZ0",
  "term_label": "Unknown biological process",
  "gene_name": "Inactive ubiquitin carboxyl-terminal hydrolase MINDY-4B"
}